{
  "gene_symbol": "TDGF1",
  "term_label": "heart development",
  "term_id": "GO:0007507",
  "gene": "UniProtKB:P13385",
  "gene_name": "Teratocarcinoma-derived growth factor 1"
}